{
  "term_id": "UNKNOWN:0001",
  "term_label": "Unknown molecular function",
  "gene_name": "TLR adapter interacting with SLC15A4 on the lysosome",
  "gene_symbol": "TASL",
  "gene": "UniProtKB:Q9HAI6"
}